{
  "gene_name": "Semaphorin-3F",
  "gene_symbol": "SEMA3F",
  "gene": "UniProtKB:Q13275",
  "term_id": "GO:0030335",
  "term_label": "positive regulation of cell migration"
}